{
  "term_id": "GO:0008630",
  "gene_name": "DNA-dependent protein kinase catalytic subunit",
  "gene": "UniProtKB:P78527",
  "term_label": "intrinsic apoptotic signaling pathway in response to DNA damage",
  "gene_symbol": "PRKDC"
}